{
  "gene": "UniProtKB:P53365",
  "term_label": "phospholipid binding",
  "gene_name": "Arfaptin-2",
  "gene_symbol": "ARFIP2",
  "term_id": "GO:0005543"
}